{
  "gene": "UniProtKB:Q8NBN3",
  "term_label": "Golgi apparatus",
  "term_id": "GO:0005794",
  "gene_symbol": "TMEM87A",
  "gene_name": "Transmembrane protein 87A"
}